{
  "term_label": "signal recognition particle binding",
  "gene_name": "Rhomboid domain-containing protein 2",
  "gene": "UniProtKB:Q6NTF9",
  "term_id": "GO:0005047",
  "gene_symbol": "RHBDD2"
}